{
  "term_id": "UNKNOWN:0002",
  "term_label": "Unknown biological process",
  "gene": "UniProtKB:Q9BZK8",
  "gene_symbol": "OCR1",
  "gene_name": "Ovarian cancer-related protein 1"
}